{
  "term_label": "sodium ion transmembrane transport",
  "gene": "UniProtKB:Q13621",
  "term_id": "GO:0035725",
  "gene_symbol": "SLC12A1",
  "gene_name": "Solute carrier family 12 member 1"
}